{
  "gene": "UniProtKB:Q6X9E4",
  "term_label": "Unknown biological process",
  "term_id": "UNKNOWN:0002",
  "gene_symbol": "FBXW12",
  "gene_name": "F-box_WD repeat-containing protein 12"
}